{
  "gene_symbol": "PPP1R16A",
  "gene_name": "Protein phosphatase 1 regulatory subunit 16A",
  "term_id": "GO:0004857",
  "term_label": "enzyme inhibitor activity",
  "gene": "UniProtKB:Q96I34"
}